{
  "gene_name": "Ret finger protein-like 4A-like protein 1",
  "gene": "UniProtKB:F8VTS6",
  "term_id": "GO:0005737",
  "gene_symbol": "RFPL4AL1",
  "term_label": "cytoplasm"
}